{
  "term_label": "regulation of transcription by RNA polymerase II",
  "gene_symbol": "LBX1",
  "term_id": "GO:0006357",
  "gene": "UniProtKB:P52954",
  "gene_name": "Transcription factor LBX1"
}